{
  "term_id": "GO:0005739",
  "term_label": "mitochondrion",
  "gene": "UniProtKB:Q5EBM0",
  "gene_name": "UMP-CMP kinase 2, mitochondrial",
  "gene_symbol": "CMPK2"
}